{
  "term_id": "GO:0000724",
  "gene_symbol": "NUCKS1",
  "term_label": "double-strand break repair via homologous recombination",
  "gene": "UniProtKB:Q9H1E3",
  "gene_name": "Nuclear ubiquitous casein and cyclin-dependent kinase substrate 1"
}